{
  "term_id": "GO:0030593",
  "gene_symbol": "LGALS3",
  "term_label": "neutrophil chemotaxis",
  "gene": "UniProtKB:P17931",
  "gene_name": "Galectin-3"
}